{
  "gene_symbol": "ZNF321P",
  "gene_name": "Putative protein ZNF321",
  "term_label": "Unknown molecular function",
  "gene": "UniProtKB:Q8N8H1",
  "term_id": "UNKNOWN:0001"
}